negative regulation of snRNA transcription by RNA polymerase II [GO:1905381] (biological process) Also known as: down regulation of snRNA transcription from Pol II promoter, down regulation of snRNA transcription from RNA polymerase II promoter, down-regulation of snRNA transcription from Pol II promoter, down-regulation of snRNA transcription from RNA polymerase II promoter, downregulation of snRNA transcription from Pol II promoter, downregulation of snRNA transcription from RNA polymerase II promoter, negative regulation of snRNA transcription from Pol II promoter, negative regulation of snRNA transcription from RNA polymerase II promoter, inhibition of snRNA transcription from Pol II promoter, inhibition of snRNA transcription from RNA polymerase II promoter Definition: Any process that stops, prevents or reduces the frequency, rate or extent of snRNA transcription mediated by RNA polymerase II. Relationships: is a type of GO:0000122; is a type of regulation of snRNA transcription by RNA polymerase II [GO:1905380]; negatively regulates GO:0042795 References: PMID:10022900 Sources: GOC:TermGenie, GOC:bhm, GO_REF:0000058